{
  "term_id": "GO:0005615",
  "gene": "UniProtKB:P10147",
  "gene_name": "C-C motif chemokine 3",
  "gene_symbol": "CCL3",
  "term_label": "extracellular space"
}